heart looping [GO:0001947] (biological process) References: PMID:12094232 Sources: GOC:dph Regulation: regulated by regulation of heart looping [GO:1901207]; negatively regulated by negative regulation of heart looping [GO:1901208]; positively regulated by GO:1901209 Relationships: is a type of embryonic heart tube morphogenesis [GO:0003143]; is part of determination of heart left/right asymmetry [GO:0061371] Definition: The tube morphogenesis process in which the primitive heart tube loops asymmetrically. This looping brings the primitive heart chambers into alignment preceding their future integration. Heart looping begins with dextral-looping and ends when the main regional divisions of the mature heart and primordium of the great arterial trunks become established preceding septation. Also known as: cardiac looping